{
  "gene_name": "RING finger protein 113B",
  "term_id": "GO:0004842",
  "gene": "UniProtKB:Q8IZP6",
  "gene_symbol": "RNF113B",
  "term_label": "ubiquitin-protein transferase activity"
}